{
  "term_id": "GO:0005543",
  "gene_symbol": "APOE",
  "gene_name": "Apolipoprotein E",
  "term_label": "phospholipid binding",
  "gene": "UniProtKB:P02649"
}